aldehyde metabolic process [GO:0006081] (biological process) Relationships: is a type of GO:0008152 Subtypes: acetaldehyde metabolic process [GO:0006117], GO:0009438, vanillin metabolic process [GO:0018982], glyceraldehyde-3-phosphate metabolic process [GO:0019682], GO:0032341, furaldehyde metabolic process [GO:0033859], retinal metabolic process [GO:0042574], pyridoxal metabolic process [GO:0042817], GO:0042822, aldehyde biosynthetic process [GO:0046184], aldehyde catabolic process [GO:0046185], formaldehyde metabolic process [GO:0046292], hexadecanal metabolic process [GO:0046458], glyoxylate metabolic process [GO:0046487], GO:0061720, glyoxal metabolic process [GO:1903189] Also known as: aldehyde metabolism, alkanal metabolic process, alkanal metabolism Sources: GOC:go_curators, ISBN:0198506732 Definition: The chemical reactions and pathways involving aldehydes, any organic compound with the formula R-CH=O, as carried out by individual cells.